{
  "term_label": "signal transduction",
  "gene_symbol": "AKAP12",
  "gene": "UniProtKB:Q02952",
  "term_id": "GO:0007165",
  "gene_name": "A-kinase anchor protein 12"
}